galacturonate biosynthetic process [GO:0033481] (biological process) Relationships: is a type of GO:0072330 Also known as: galacturonate anabolism, galacturonate biosynthesis, galacturonate formation, galacturonate synthesis Subtypes: GO:0033482 Sources: GOC:mah Definition: The chemical reactions and pathways resulting in the formation of galacturonate, the anion of galacturonic acid.